receptor clustering [GO:0043113] (biological process) Relationships: is a type of GO:0072657; occurs in plasma membrane [GO:0005886] Subtypes: ciliary receptor clustering involved in smoothened signaling pathway [GO:0060830], skeletal muscle acetylcholine-gated channel clustering [GO:0071340], neurotransmitter-gated ion channel clustering [GO:0072578], neurexin clustering involved in presynaptic membrane assembly [GO:0097115], neuroligin clustering involved in postsynaptic membrane assembly [GO:0097118] References: PMID:19747931, PMID:21453460 Sources: GOC:bf, GOC:jl, GOC:pr Definition: The receptor metabolic process that results in grouping of a set of receptors at a cellular location, often to amplify the sensitivity of a signaling response. Regulation: regulated by GO:1903909; negatively regulated by negative regulation of receptor clustering [GO:1903910]; positively regulated by positive regulation of receptor clustering [GO:1903911]